{
  "term_label": "PML body",
  "gene_symbol": "KLHL20",
  "gene_name": "Kelch-like protein 20",
  "term_id": "GO:0016605",
  "gene": "UniProtKB:Q9Y2M5"
}